saccharopine oxidase activity [GO:0051698] (molecular function) References: PMID:16233628 Sources: RHEA:28210 Also known as: SAX activity Relationships: is a type of oxidoreductase activity, acting on the CH-NH group of donors, oxygen as acceptor [GO:0016647] Definition: Catalysis of the reaction: H2O + L-saccharopine + O2 = (S)-2-amino-6-oxohexanoate + H2O2 + L-glutamate.